cell wall macromolecule catabolic process involved in fungal-type cell wall disassembly [GO:0071854] (biological process) Definition: The chemical reactions and pathways that result in the breakdown of macromolecules that form part of a cell wall, and contributes to the breakdown of the fungal-type cell wall. Relationships: is a type of cell wall macromolecule catabolic process involved in cell wall disassembly [GO:0070910]; is part of fungal-type cell wall disassembly [GO:0071853] Sources: GOC:mah